{
  "term_label": "Unknown cellular component",
  "gene_name": "T cell receptor alpha variable 10",
  "gene_symbol": "TRAV10",
  "gene": "UniProtKB:A0A0B4J240",
  "term_id": "UNKNOWN:0003"
}